{
  "gene_name": "BSD domain-containing protein 1",
  "term_id": "UNKNOWN:0001",
  "term_label": "Unknown molecular function",
  "gene_symbol": "BSDC1",
  "gene": "UniProtKB:Q9NW68"
}